{
  "term_label": "lipid catabolic process",
  "gene": "UniProtKB:Q8WWY8",
  "gene_symbol": "LIPH",
  "gene_name": "Lipase member H",
  "term_id": "GO:0016042"
}